{
  "gene_name": "Enhancer of mRNA-decapping protein 4",
  "term_label": "Unknown molecular function",
  "gene_symbol": "EDC4",
  "gene": "UniProtKB:Q6P2E9",
  "term_id": "UNKNOWN:0001"
}